{
  "term_id": "GO:0050431",
  "gene": "UniProtKB:Q6EMK4",
  "gene_symbol": "VASN",
  "gene_name": "Vasorin",
  "term_label": "transforming growth factor beta binding"
}